{
  "term_label": "Unknown biological process",
  "gene_name": "Bone marrow proteoglycan",
  "gene": "UniProtKB:P13727",
  "gene_symbol": "PRG2",
  "term_id": "UNKNOWN:0002"
}